{
  "gene_name": "Putative uncharacterized protein FRMD6-AS1",
  "term_id": "UNKNOWN:0003",
  "term_label": "Unknown cellular component",
  "gene_symbol": "FRMD6-AS1",
  "gene": "UniProtKB:P0C7T7"
}